puncta adhaerentia [GO:0044288] (cellular component) Relationships: is a type of zonula adherens [GO:0005915] Definition: A small version of the zonula adherens type junction, characterized by a symmetrical adherent point between two cells. Sources: NIF_Subcellular:sao257629430